{
  "term_id": "GO:0035556",
  "gene_name": "Amyloid beta A4 precursor protein-binding family B member 1-interacting protein",
  "term_label": "intracellular signal transduction",
  "gene": "UniProtKB:Q7Z5R6",
  "gene_symbol": "APBB1IP"
}